{
  "gene_name": "von Willebrand factor A domain-containing protein 5A",
  "term_label": "Unknown biological process",
  "gene": "UniProtKB:O00534",
  "term_id": "UNKNOWN:0002",
  "gene_symbol": "VWA5A"
}